{
  "gene": "UniProtKB:Q53H47",
  "term_label": "replication fork processing",
  "gene_name": "Histone-lysine N-methyltransferase SETMAR",
  "gene_symbol": "SETMAR",
  "term_id": "GO:0031297"
}